{
  "term_label": "epidermal growth factor receptor binding",
  "gene": "UniProtKB:Q99075",
  "term_id": "GO:0005154",
  "gene_name": "Proheparin-binding EGF-like growth factor",
  "gene_symbol": "HBEGF"
}